{
  "gene_name": "Raftlin-2",
  "gene_symbol": "RFTN2",
  "gene": "UniProtKB:Q52LD8",
  "term_id": "UNKNOWN:0002",
  "term_label": "Unknown biological process"
}